{
  "term_id": "GO:0001817",
  "gene": "UniProtKB:Q7KYR7",
  "gene_symbol": "BTN2A1",
  "gene_name": "Butyrophilin subfamily 2 member A1",
  "term_label": "regulation of cytokine production"
}